sclerotium development [GO:1990045] (biological process) Definition: The process whose specific outcome is the progression of the sclerotium over time, from its formation to the mature structure. A sclerotium is a mycelial resting body, resistant to adverse environmental conditions. References: PMID:21148914 Sources: GOC:di Relationships: is a type of GO:0048856 Regulation: regulated by regulation of sclerotium development [GO:1901922]; negatively regulated by negative regulation of sclerotium development [GO:1901923]; positively regulated by positive regulation of sclerotium development [GO:1901924]